{
  "gene": "UniProtKB:Q5PRF9",
  "term_id": "GO:0000289",
  "term_label": "nuclear-transcribed mRNA poly(A) tail shortening",
  "gene_name": "Protein Smaug homolog 2",
  "gene_symbol": "SAMD4B"
}